{
  "gene_symbol": "LOC122513141",
  "term_label": "proteasome-mediated ubiquitin-dependent protein catabolic process",
  "gene_name": "RING-type domain-containing protein",
  "term_id": "GO:0043161",
  "gene": "UniProtKB:A0A2R8Y4M4"
}